apolipoprotein A-I-mediated signaling pathway [GO:0038027] (biological process) Also known as: apolipoprotein A-I-mediated signalling pathway References: PMID:16443932 Sources: GOC:bf, GOC:signaling Regulation: regulated by regulation of apolipoprotein A-I-mediated signaling pathway [GO:1905094]; negatively regulated by negative regulation of apolipoprotein A-I-mediated signaling pathway [GO:1905095]; positively regulated by positive regulation of apolipoprotein A-I-mediated signaling pathway [GO:1905096] Relationships: is a type of cell surface receptor signaling pathway [GO:0007166] Definition: The series of molecular signals initiated by apolipoprotein A-I binding to its receptor on the surface of a target cell, and ending with the regulation of a downstream cellular process, e.g. transcription.